agglutination involved in conjugation with cellular fusion [GO:0000752] (biological process) Relationships: is a type of biological process involved in intraspecies interaction between organisms [GO:0051703]; is a type of cell-cell adhesion in response to extracellular stimulus [GO:0140039]; is part of conjugation with cellular fusion [GO:0000747]; is part of response to pheromone triggering conjugation with cellular fusion [GO:0000749] Also known as: agglutination, cell-cell adhesion during conjugation with cellular fusion, cell-cell adhesion during mating Definition: The aggregation or adhesion of compatible mating types via complementary cell-cell interactions during conjugation with cellular fusion of a unicellular organism. An example of this process is agglutination in Saccharomyces cerevisiae. Sources: GOC:elh